{
  "gene": "UniProtKB:Q7Z7B0",
  "gene_symbol": "FILIP1",
  "gene_name": "Filamin-A-interacting protein 1",
  "term_id": "GO:1903119",
  "term_label": "protein localization to actin cytoskeleton"
}